{
  "gene_name": "Tubulin polymerization-promoting protein",
  "gene_symbol": "TPPP",
  "term_id": "GO:0005874",
  "term_label": "microtubule",
  "gene": "UniProtKB:O94811"
}